{
  "gene": "UniProtKB:Q9P283",
  "gene_name": "Semaphorin-5B",
  "term_label": "axon guidance",
  "gene_symbol": "SEMA5B",
  "term_id": "GO:0007411"
}